{
  "term_label": "extracellular space",
  "gene_name": "Angiotensinogen",
  "gene": "UniProtKB:P01019",
  "term_id": "GO:0005615",
  "gene_symbol": "AGT"
}